{
  "term_id": "GO:0000978",
  "gene_name": "Zinc finger protein 419",
  "gene_symbol": "ZNF419",
  "gene": "UniProtKB:Q96HQ0",
  "term_label": "RNA polymerase II cis-regulatory region sequence-specific DNA binding"
}